{
  "term_label": "Unknown cellular component",
  "term_id": "UNKNOWN:0003",
  "gene": "UniProtKB:Q8IYK4",
  "gene_symbol": "COLGALT2",
  "gene_name": "Procollagen galactosyltransferase 2"
}